{
  "term_label": "olfactory receptor activity",
  "gene": "UniProtKB:Q8NGZ3",
  "gene_symbol": "OR13G1",
  "term_id": "GO:0004984",
  "gene_name": "Olfactory receptor 13G1"
}